{
  "gene": "UniProtKB:Q9NWB7",
  "gene_symbol": "IFT57",
  "term_id": "GO:0005815",
  "term_label": "microtubule organizing center",
  "gene_name": "Intraflagellar transport protein 57 homolog"
}